viral translational shunt [GO:0039704] (biological process) Definition: A viral translation initiation mechanism where ribosomes are loaded onto viral mRNA at the 5'-cap structure and start scanning for a short distance before by-passing the large internal leader region and initiating at a downstream start site. Also known as: ribosomal shunt initiation pathway Relationships: is a type of viral translation [GO:0019081] References: PMID:15827182, PMID:18195037 Sources: VZ:608 Note: This term is intended to annotate gene products involved in the process of viral translational shunt, not viral proteins produced by this translation process.